{
  "gene": "UniProtKB:Q9BVG3",
  "gene_symbol": "TRIM62",
  "gene_name": "E3 ubiquitin-protein ligase TRIM62",
  "term_id": "GO:0005737",
  "term_label": "cytoplasm"
}